methyl jasmonate esterase activity [GO:0080032] (molecular function) Relationships: is a type of GO:0052689 Definition: Catalysis of the reaction: H2O + methyl (-)-jasmonate = H+ + jasmonate + methanol. Also known as: MEJA esterase activity, jasmonic acid methyl ester esterase activity, methyl JA esterase activity References: PMID:15233793, PMID:18467465 Sources: RHEA:55372